{
  "gene": "UniProtKB:Q92673",
  "term_id": "GO:0006622",
  "gene_symbol": "SORL1",
  "gene_name": "Sortilin-related receptor",
  "term_label": "protein targeting to lysosome"
}